{
  "gene_symbol": "PSMA3",
  "gene_name": "Proteasome subunit alpha type-3",
  "term_id": "UNKNOWN:0001",
  "term_label": "Unknown molecular function",
  "gene": "UniProtKB:P25788"
}